{
  "gene": "UniProtKB:Q8N8Q3",
  "term_label": "nucleolus",
  "gene_name": "Endonuclease V",
  "gene_symbol": "ENDOV",
  "term_id": "GO:0005730"
}